cellular response to nonylphenol [GO:1904148] (biological process) Definition: Any process that results in a change in state or activity of a cell (in terms of movement, secretion, enzyme production, gene expression, etc.) as a result of a nonylphenol stimulus. Relationships: is a type of GO:0070887; is a type of response to nonylphenol [GO:1904147] References: PMID:19260726 Sources: GOC:TermGenie, GO_REF:0000071